{
  "term_id": "GO:0035198",
  "term_label": "miRNA binding",
  "gene_name": "Protein argonaute-1",
  "gene_symbol": "AGO1",
  "gene": "UniProtKB:Q9UL18"
}